{
  "gene": "UniProtKB:Q8WZ59",
  "term_label": "Unknown molecular function",
  "term_id": "UNKNOWN:0001",
  "gene_symbol": "TMEM190",
  "gene_name": "Transmembrane protein 190"
}